regulates [RO:0002211] (external)